{
  "term_id": "GO:0071011",
  "term_label": "precatalytic spliceosome",
  "gene_name": "Splicing factor 3B subunit 2",
  "gene_symbol": "SF3B2",
  "gene": "UniProtKB:Q13435"
}